{
  "term_id": "UNKNOWN:0003",
  "gene_symbol": "NT5DC1",
  "gene": "UniProtKB:Q5TFE4",
  "term_label": "Unknown cellular component",
  "gene_name": "5'-nucleotidase domain-containing protein 1"
}